{
  "gene": "UniProtKB:Q9BXG8",
  "term_label": "Unknown molecular function",
  "term_id": "UNKNOWN:0001",
  "gene_name": "Spermatogenic leucine zipper protein 1",
  "gene_symbol": "SPZ1"
}